{
  "term_label": "lysosomal membrane",
  "gene_symbol": "HLA-DPB1",
  "gene_name": "HLA class II histocompatibility antigen, DP beta 1 chain",
  "term_id": "GO:0005765",
  "gene": "UniProtKB:P04440"
}